{
  "term_id": "GO:0008047",
  "term_label": "enzyme activator activity",
  "gene_symbol": "DAOA",
  "gene_name": "D-amino acid oxidase activator",
  "gene": "UniProtKB:P59103"
}